{
  "gene_symbol": "TRAPPC2B",
  "term_id": "GO:0005737",
  "gene_name": "Trafficking protein particle complex subunit 2B",
  "gene": "UniProtKB:P0DI82",
  "term_label": "cytoplasm"
}